{
  "gene": "UniProtKB:P47874",
  "gene_symbol": "OMP",
  "term_id": "GO:0043025",
  "gene_name": "Olfactory marker protein",
  "term_label": "neuronal cell body"
}